{
  "gene_symbol": "DYNLRB1",
  "gene": "UniProtKB:Q9NP97",
  "term_label": "cytoplasm",
  "gene_name": "Dynein light chain roadblock-type 1",
  "term_id": "GO:0005737"
}